{
  "term_label": "cellular response to insulin stimulus",
  "gene_symbol": "INSIG1",
  "term_id": "GO:0032869",
  "gene_name": "Insulin-induced gene 1 protein",
  "gene": "UniProtKB:O15503"
}